{
  "gene_symbol": "A0A1W2PPM0",
  "gene": "UniProtKB:A0A1W2PPM0",
  "gene_name": "Uncharacterized protein",
  "term_id": "UNKNOWN:0002",
  "term_label": "Unknown biological process"
}